motor learning [GO:0061743] (biological process) Definition: Any process in which an organism acquires a novel neuromuscular action or movement as the result of experience. Sources: GOC:PARL, GOC:bf, Wikipedia:Motor_learning Relationships: is a type of learning [GO:0007612]